{
  "gene_symbol": "CRY2",
  "gene_name": "Cryptochrome-2",
  "term_label": "negative regulation of DNA-templated transcription",
  "term_id": "GO:0045892",
  "gene": "UniProtKB:Q49AN0"
}